beta-pyrazolylalanine synthase activity [GO:0047458] (molecular function) Also known as: beta-pyrazolylalanine synthase (acetylserine) activity, 3-O-acetyl-L-serine:pyrazole 1-(2-amino-2-carboxyethyl)transferase activity, BPA-synthase activity, O(3)-acetyl-L-serine acetate-lyase (adding pyrazole) activity, O3-acetyl-L-serine acetate-lyase (adding pyrazole), O3-acetyl-L-serine:pyrazole 1-(2-amino-2-carboxyethyl)transferase activity, beta-(1-pyrazolyl)alanine synthase activity, beta-pyrazolealanine synthase activity, pyrazolealanine synthase activity, pyrazolylalaninase activity Sources: RHEA:13117 Definition: Catalysis of the reaction: O-acetyl-L-serine + pyrazole = 3-(pyrazol-1-yl)-L-alanine + acetate + H+. Relationships: is a type of transferase activity, transferring alkyl or aryl (other than methyl) groups [GO:0016765]